{
  "gene_name": "RING finger protein 151",
  "term_id": "GO:0061630",
  "term_label": "ubiquitin protein ligase activity",
  "gene": "UniProtKB:Q2KHN1",
  "gene_symbol": "RNF151"
}